{
  "gene_symbol": "SRC",
  "term_label": "epidermal growth factor receptor signaling pathway",
  "gene": "UniProtKB:P12931",
  "gene_name": "Proto-oncogene tyrosine-protein kinase Src",
  "term_id": "GO:0007173"
}